{
  "gene": "UniProtKB:P58004",
  "term_label": "Unknown cellular component",
  "gene_name": "Sestrin-2",
  "gene_symbol": "SESN2",
  "term_id": "UNKNOWN:0003"
}